{
  "gene_name": "CTTNBP2 N-terminal-like protein",
  "term_id": "GO:0015629",
  "gene": "UniProtKB:Q9P2B4",
  "gene_symbol": "CTTNBP2NL",
  "term_label": "actin cytoskeleton"
}